establishment of lymphocyte polarity [GO:0001767] (biological process) Definition: The directed orientation of lymphocyte signaling molecules and associated membrane rafts towards a chemokine gradient or a contact point with an appropriate activating cell. Also known as: lymphocyte polarization Relationships: is a type of GO:0030010; is part of GO:0046649 Subtypes: GO:0001768, establishment of B cell polarity [GO:0001769], establishment of natural killer cell polarity [GO:0001770] References: PMID:11244041, PMID:12615889 Sources: GOC:mgi_curators